{
  "gene_name": "Glutathione reductase, mitochondrial",
  "term_label": "flavin adenine dinucleotide binding",
  "gene_symbol": "GSR",
  "term_id": "GO:0050660",
  "gene": "UniProtKB:P00390"
}